{
  "gene": "UniProtKB:P35527",
  "gene_symbol": "KRT9",
  "gene_name": "Keratin, type I cytoskeletal 9",
  "term_label": "cytoskeleton",
  "term_id": "GO:0005856"
}